{
  "gene_symbol": "BRSK2",
  "gene_name": "Serine_threonine-protein kinase BRSK2",
  "term_id": "GO:0005813",
  "gene": "UniProtKB:Q8IWQ3",
  "term_label": "centrosome"
}